{
  "term_id": "GO:0005085",
  "gene_name": "Ras-specific guanine nucleotide-releasing factor 2",
  "gene": "UniProtKB:O14827",
  "gene_symbol": "RASGRF2",
  "term_label": "guanyl-nucleotide exchange factor activity"
}